{
  "gene_symbol": "GOLGA8CP",
  "term_label": "Unknown molecular function",
  "gene_name": "Golgin subfamily A member 8C",
  "gene": "UniProtKB:A6NN73",
  "term_id": "UNKNOWN:0001"
}